{
  "gene_name": "Leukocyte-specific transcript 1 protein",
  "term_id": "GO:0016358",
  "gene": "UniProtKB:O00453",
  "gene_symbol": "LST1",
  "term_label": "dendrite development"
}